{
  "gene_name": "BAH and coiled-coil domain-containing protein 1",
  "term_label": "Unknown molecular function",
  "gene_symbol": "BAHCC1",
  "gene": "UniProtKB:Q9P281",
  "term_id": "UNKNOWN:0001"
}